fatty acid beta-oxidation, unsaturated, even number, epimerase pathway [GO:0033544] (biological process) Sources: GOC:mah, MetaCyc:PWY-5138 Definition: A fatty acid beta-oxidation pathway by which fatty acids having cis-double bonds on even-numbered carbons are degraded. In this pathway, the intermediate 2,4-dienoyl-CoA is converted to cis-2-enoyl-CoA through one more cycle of the core beta-oxidation pathway. Cis-2-enoyl-CoA cannot be completely degraded via the core beta-oxidation pathway because hydratation of cis-2-enoyl-CoA yields D-3-hydroxyacyl-CoA, which is not a substrate for 3-hydroxylacyl-CoA dehydrogenase. Cis-2-enoyl-CoA must enter the so-called epimerase pathway, which involves converting D-3-hydroxyacyl-CoA to L-3-hydroxyacyl-CoA by 3-hydroxylacyl-CoA epimerase or by two stereo-specific enoyl-CoA hydratases. L-3-hydroxyacyl-CoA then returns to the core beta-oxidation pathway. Fatty acid beta-oxidation begins with the addition of coenzyme A to a fatty acid, and ends when only two or three carbons remain (as acetyl-CoA or propionyl-CoA respectively). Relationships: is a type of fatty acid beta-oxidation, unsaturated, even number [GO:0033542]